{
  "gene_name": "Disintegrin and metalloproteinase domain-containing protein 18",
  "gene_symbol": "ADAM18",
  "term_id": "GO:0007339",
  "term_label": "binding of sperm to zona pellucida",
  "gene": "UniProtKB:Q9Y3Q7"
}